negative regulation of substance P secretion, neurotransmission [GO:1904495] (biological process) Definition: Any process that stops, prevents or reduces the frequency, rate or extent of substance P secretion, neurotransmission. References: PMID:15292051 Sources: GOC:TermGenie, GO_REF:0000058 Also known as: down regulation of substance P secretion, neurotransmission, down-regulation of substance P secretion, neurotransmission, downregulation of substance P secretion, neurotransmission, inhibition of substance P secretion, neurotransmission Relationships: is a type of negative regulation of neurotransmitter secretion [GO:0046929]; is a type of GO:1904459; is a type of regulation of substance P secretion, neurotransmission [GO:1904494]; negatively regulates substance P secretion, neurotransmission [GO:1990793]